{
  "term_label": "Unknown biological process",
  "term_id": "UNKNOWN:0002",
  "gene": "UniProtKB:Q7Z5L7",
  "gene_symbol": "PODN",
  "gene_name": "Podocan"
}